wound healing involved in inflammatory response [GO:0002246] (biological process) Relationships: is a type of wound healing [GO:0042060]; is part of inflammatory response to wounding [GO:0090594] Sources: GOC:jal, ISBN:0721601871 Definition: The series of events that restore integrity to damaged tissue that contribute to an inflammatory response. Also known as: healing during inflammatory response, inflammatory response wound healing